{
  "term_id": "GO:0001756",
  "term_label": "somitogenesis",
  "gene_symbol": "TBX18",
  "gene_name": "T-box transcription factor TBX18",
  "gene": "UniProtKB:O95935"
}